{
  "gene_symbol": "FLRT2",
  "term_label": "Unknown biological process",
  "gene_name": "Leucine-rich repeat transmembrane protein FLRT2",
  "gene": "UniProtKB:O43155",
  "term_id": "UNKNOWN:0002"
}